ferric-chelate reductase (NADH) activity [GO:0140618] (molecular function) Also known as: ferric chelate reductase activity, iron chelate reductase activity, NADH:Fe(3+) oxidoreductase activity, NADH:Fe3+ oxidoreductase activity Sources: RHEA:15061 Relationships: is a type of ferric-chelate reductase activity [GO:0000293]; is a type of oxidoreductase activity, acting on metal ions, NAD or NADP as acceptor [GO:0016723] Definition: Catalysis of the reaction: 2 a Fe(II)-siderophore + NAD+ + H+ = 2 a Fe(III)-siderophore + NADH.